{
  "gene": "UniProtKB:P48539",
  "gene_symbol": "PCP4",
  "term_label": "cytoplasm",
  "term_id": "GO:0005737",
  "gene_name": "Calmodulin regulator protein PCP4"
}